endosome membrane tubulation [GO:0097750] (biological process) References: PMID:26911690 Sources: GOC:PARL, GOC:bc Definition: A membrane tubulation process occurring in an endosome membrane. Also known as: endosomal membrane tubulation Relationships: is a type of endosome organization [GO:0007032]; is a type of membrane tubulation [GO:0097749]